wobble position guanine ribose methylation [GO:0002129] (biological process) Relationships: is a type of GO:0002130; is_a tRNA guanine ribose methylation [GO:0002938] Definition: The process in which the ribose of guanosine at position 34 in the anticodon of a tRNA is post-transcriptionally methylated at the 2'-O position. Sources: GOC:hjd, ISBN:155581073X